{
  "gene_name": "T cell receptor beta variable 4-1",
  "term_label": "cell surface receptor signaling pathway",
  "gene_symbol": "TRBV4-1",
  "term_id": "GO:0007166",
  "gene": "UniProtKB:A0A577"
}